{
  "gene_symbol": "CDK12",
  "gene": "UniProtKB:Q9NYV4",
  "term_id": "GO:0032968",
  "gene_name": "Cyclin-dependent kinase 12",
  "term_label": "positive regulation of transcription elongation by RNA polymerase II"
}